{
  "gene": "UniProtKB:Q9Y6F9",
  "term_id": "GO:0005109",
  "gene_name": "Protein Wnt-6",
  "gene_symbol": "WNT6",
  "term_label": "frizzled binding"
}